{
  "term_id": "GO:0004984",
  "gene_symbol": "OR6B1",
  "gene_name": "Olfactory receptor 6B1",
  "term_label": "olfactory receptor activity",
  "gene": "UniProtKB:O95007"
}